hydrolase activity, acting on acid sulfur-sulfur bonds [GO:0016828] (molecular function) Definition: Catalysis of the hydrolysis of any acid sulfur-sulfur bond. Also known as: hydrolase activity, acting on acid sulphur-sulphur bonds Relationships: is a type of hydrolase activity [GO:0016787] Subtypes: trithionate hydrolase activity [GO:0047401] Sources: EC:3.12.-.-